negative regulation of synaptic vesicle uncoating [GO:1903389] (biological process) Relationships: is a type of negative regulation of synaptic vesicle endocytosis [GO:1900243]; is a type of negative regulation of protein depolymerization [GO:1901880]; is a type of regulation of synaptic vesicle uncoating [GO:1903388]; negatively regulates GO:0016191 Also known as: down regulation of synaptic vesicle coat depolymerization, down regulation of synaptic vesicle coat protein depolymerization, down regulation of synaptic vesicle uncoating, down-regulation of synaptic vesicle coat depolymerization, down-regulation of synaptic vesicle coat protein depolymerization, down-regulation of synaptic vesicle uncoating, downregulation of synaptic vesicle coat depolymerization, downregulation of synaptic vesicle coat protein depolymerization, downregulation of synaptic vesicle uncoating, negative regulation of synaptic vesicle coat depolymerization, negative regulation of synaptic vesicle coat protein depolymerization, inhibition of synaptic vesicle coat depolymerization, inhibition of synaptic vesicle coat protein depolymerization, inhibition of synaptic vesicle uncoating References: PMID:21563316 Sources: GOC:PARL, GOC:TermGenie, GOC:pad, GO_REF:0000058 Definition: Any process that stops, prevents or reduces the frequency, rate or extent of synaptic vesicle uncoating.